{
  "gene": "UniProtKB:P51692",
  "gene_name": "Signal transducer and activator of transcription 5B",
  "term_label": "defense response",
  "gene_symbol": "STAT5B",
  "term_id": "GO:0006952"
}